hair follicle development [GO:0001942] (biological process) Regulation: regulated by regulation of hair follicle development [GO:0051797]; RO_0002213 by positive regulation of hair follicle development [GO:0051798]; negatively regulated by negative regulation of hair follicle development [GO:0051799] Relationships: is a type of hair cycle process [GO:0022405]; is a type of anatomical structure development [GO:0048856]; is part of skin epidermis development [GO:0098773] Sources: GOC:dph, UBERON:0002073 Definition: The process whose specific outcome is the progression of the hair follicle over time, from its formation to the mature structure. A hair follicle is a tube-like opening in the epidermis where the hair shaft develops and into which the sebaceous glands open.